{
  "term_id": "GO:0034045",
  "term_label": "phagophore assembly site membrane",
  "gene_name": "Serine_threonine-protein kinase ULK3",
  "gene": "UniProtKB:Q6PHR2",
  "gene_symbol": "ULK3"
}